{
  "gene": "UniProtKB:Q8N8W4",
  "gene_name": "Omega-hydroxyceramide transacylase",
  "gene_symbol": "PNPLA1",
  "term_label": "membrane",
  "term_id": "GO:0016020"
}